{
  "gene_name": "Aminomethyltransferase, mitochondrial",
  "term_label": "glycine decarboxylation via glycine cleavage system",
  "gene_symbol": "AMT",
  "term_id": "GO:0019464",
  "gene": "UniProtKB:P48728"
}